{
  "gene_name": "Glutaredoxin-3",
  "term_id": "GO:0005634",
  "gene_symbol": "GLRX3",
  "gene": "UniProtKB:O76003",
  "term_label": "nucleus"
}